{
  "gene_name": "RING-type E3 ubiquitin-protein ligase PPIL2",
  "term_id": "GO:0061630",
  "gene": "UniProtKB:Q13356",
  "term_label": "ubiquitin protein ligase activity",
  "gene_symbol": "PPIL2"
}